{
  "gene_symbol": "A0A2R8Y4M2",
  "gene_name": "Uncharacterized protein",
  "term_id": "UNKNOWN:0003",
  "gene": "UniProtKB:A0A2R8Y4M2",
  "term_label": "Unknown cellular component"
}